N2-acetyl-L-aminoadipate kinase activity [GO:0043744] (molecular function) Definition: Catalysis of the reaction: ATP + N-acetyl-L-2-aminoadipate = ADP + N-acetyl-L-2-aminoadipate 6-phosphate. References: PMID:25392000, PMID:26966182 Sources: RHEA:41944 Relationships: is a type of phosphotransferase activity, carboxyl group as acceptor [GO:0016774]; is a type of amino acid kinase activity [GO:0019202] Also known as: N-acetyl-L-aminoadipate 5-phosphotransferase activity, N-acetylaminoadipate kinase activity, acetylaminoadipate kinase activity, [LysW]-aminoadipate kinase